{
  "gene": "UniProtKB:Q96EW2",
  "gene_name": "HSPB1-associated protein 1",
  "term_label": "Unknown biological process",
  "term_id": "UNKNOWN:0002",
  "gene_symbol": "HSPBAP1"
}